positive regulation of histamine secretion by mast cell [GO:1903595] (biological process) Definition: Any process that activates or increases the frequency, rate or extent of histamine secretion by mast cell. References: PMID:18253931 Sources: GOC:TermGenie, GOC:als, GO_REF:0000058 Relationships: is a type of GO:0043306; is a type of positive regulation of hormone secretion [GO:0046887]; is a type of positive regulation of inflammatory response [GO:0050729]; is_a GO:0051240; is a type of GO:1903593; RO_0002213 GO:0002553 Also known as: up regulation of histamine secretion by mast cell, up-regulation of histamine secretion by mast cell, upregulation of histamine secretion by mast cell, activation of histamine secretion by mast cell